{
  "gene_name": "Lysosomal acid lipase_cholesteryl ester hydrolase",
  "gene": "UniProtKB:P38571",
  "term_id": "UNKNOWN:0003",
  "gene_symbol": "LIPA",
  "term_label": "Unknown cellular component"
}